3-hydroxy-2-methylpyridine-4,5-dicarboxylate 4-decarboxylase activity [GO:0047431] (molecular function) Definition: Catalysis of the reaction: 5-hydroxy-6-methylpyridine-3,4-dicarboxylate + H+ = 5-hydroxy-6-methylpyridine-3-carboxylate + CO2. Relationships: is a type of carboxy-lyase activity [GO:0016831] Sources: EC:4.1.1.51, RHEA:13669 Also known as: 3-hydroxy-2-methylpyridine-4,5-dicarboxylate 4-carboxy-lyase (3-hydroxy-2-methylpyridine-5-carboxylate-forming), 3-hydroxy-2-methylpyridine-4,5-dicarboxylate 4-carboxy-lyase activity